{
  "gene": "UniProtKB:Q9HBM0",
  "gene_name": "Vezatin",
  "term_id": "UNKNOWN:0001",
  "term_label": "Unknown molecular function",
  "gene_symbol": "VEZT"
}